{
  "gene": "UniProtKB:P36542",
  "gene_name": "ATP synthase subunit gamma, mitochondrial",
  "term_id": "GO:0046933",
  "term_label": "proton-transporting ATP synthase activity, rotational mechanism",
  "gene_symbol": "ATP5F1C"
}